interleukin-15 binding [GO:0042009] (molecular function) Also known as: IL-15 binding Relationships: is a type of cytokine binding [GO:0019955] Definition: Binding to interleukin-15. Sources: GOC:jl